{
  "term_label": "lysosome",
  "gene_symbol": "RRAGD",
  "gene_name": "Ras-related GTP-binding protein D",
  "term_id": "GO:0005764",
  "gene": "UniProtKB:Q9NQL2"
}